{
  "term_label": "membrane",
  "gene_symbol": "KCNA4",
  "term_id": "GO:0016020",
  "gene": "UniProtKB:P22459",
  "gene_name": "Potassium voltage-gated channel subfamily A member 4"
}